regulation of retrograde trans-synaptic signaling by neuropeptide [GO:1905432] (biological process) References: PMID:19448629 Sources: GOC:PARL, GOC:TermGenie, GOC:bf, GO_REF:0000058 Definition: Any process that modulates the frequency, rate or extent of retrograde trans-synaptic signaling by neuropeptide. Also known as: regulation of neuropeptide-mediated retrograde trans-synaptic signaling Subtypes: negative regulation of retrograde trans-synaptic signaling by neuropeptide [GO:1905433], positive regulation of retrograde trans-synaptic signaling by neuropeptide [GO:1905434] Relationships: is a type of regulation of trans-synaptic signaling [GO:0099177]; regulates GO:0099082